sulfation [GO:0051923] (biological process) Subtypes: GO:0006477 Definition: The addition of a sulfate group to a molecule. Sources: Wikipedia:Sulfation Relationships: is a type of sulfur compound metabolic process [GO:0006790] Also known as: phase II metabolism, sulfonation, sulfur addition, sulphation, sulphur addition